{
  "term_label": "Unknown biological process",
  "gene_name": "Uncharacterized protein",
  "gene_symbol": "A0A8Q3WLD3",
  "term_id": "UNKNOWN:0002",
  "gene": "UniProtKB:A0A8Q3WLD3"
}